glutamate dehydrogenase (NAD+) activity [GO:0004352] (molecular function) Note: Note that this term has a MetaCyc pathway reference as the pathway only has a single step. Also known as: L-glutamate dehydrogenase, glutamic acid dehydrogenase, glutamic dehydrogenase activity, L-glutamate:NAD+ oxidoreductase (deaminating), NAD-dependent glutamate dehydrogenase activity, NAD-dependent glutamic dehydrogenase activity, NAD-glutamate dehydrogenase activity, NAD-linked glutamate dehydrogenase activity, NAD-linked glutamic dehydrogenase activity, NAD-specific glutamate dehydrogenase activity, NAD-specific glutamic dehydrogenase activity, NAD:glutamate oxidoreductase activity, NADH-linked glutamate dehydrogenase activity, glutamate dehydrogenase (NAD), glutamate oxidoreductase activity Sources: EC:1.4.1.2 Definition: Catalysis of the reaction: L-glutamate + H2O + NAD+ = 2-oxoglutarate + NH3 + NADH + H+. Relationships: is a type of GO:0004353